glyceraldehyde oxidoreductase activity [GO:0043795] (molecular function) Definition: Catalysis of the reaction: A + D-glyceraldehyde + H2O = (R)-glycerate + AH2 + H+. Relationships: is a type of oxidoreductase activity, acting on the aldehyde or oxo group of donors [GO:0016903] References: PMID:10095793 Sources: RHEA:36047